positive regulation of isotype switching to IgG isotypes [GO:0048304] (biological process) Sources: GOC:jid Also known as: positive regulation of class switch recombination to IgG isotypes, positive regulation of class switching to IgG isotypes, positive regulation of isotype switch recombination to IgG isotypes, up regulation of isotype switching to IgG isotypes, up-regulation of isotype switching to IgG isotypes, upregulation of isotype switching to IgG isotypes, activation of isotype switching to IgG isotypes, stimulation of isotype switching to IgG isotypes Relationships: is a type of positive regulation of isotype switching [GO:0045830]; is a type of regulation of isotype switching to IgG isotypes [GO:0048302]; positively regulates isotype switching to IgG isotypes [GO:0048291] Definition: Any process that activates or increases the frequency, rate or extent of isotype switching to IgG isotypes.